{
  "gene": "UniProtKB:P02533",
  "term_label": "structural constituent of skin epidermis",
  "term_id": "GO:0030280",
  "gene_name": "Keratin, type I cytoskeletal 14",
  "gene_symbol": "KRT14"
}